{
  "term_label": "BORC complex",
  "term_id": "GO:0099078",
  "gene_symbol": "BLOC1S2",
  "gene": "UniProtKB:Q6QNY1",
  "gene_name": "Biogenesis of lysosome-related organelles complex 1 subunit 2"
}